Fc-gamma receptor signaling pathway involved in phagocytosis [GO:0038096] (biological process) Regulation: regulated by regulation of Fc-gamma receptor signaling pathway involved in phagocytosis [GO:1905449]; negatively regulated by negative regulation of Fc-gamma receptor signaling pathway involved in phagocytosis [GO:1905450]; positively regulated by GO:1905451 References: PMID:12488490, PMID:15466916 Sources: GOC:phg Relationships: is_a GO:0002431; is a type of immune response-regulating cell surface receptor signaling pathway involved in phagocytosis [GO:0002433]; is a type of GO:0038094 Definition: An Fc-gamma receptor signaling pathway that contributes to the endocytic engulfment of external particulate material by phagocytes. Also known as: Fc gamma receptor-dependent phagocytosis, Fc-gamma receptor signalling pathway involved in phagocytosis, Fcgamma receptor-mediated phagocytosis, IgG-mediated phagocytosis